{
  "gene": "UniProtKB:O60636",
  "gene_symbol": "TSPAN2",
  "term_label": "Unknown molecular function",
  "term_id": "UNKNOWN:0001",
  "gene_name": "Tetraspanin-2"
}